{
  "term_label": "retrograde vesicle-mediated transport, Golgi to endoplasmic reticulum",
  "gene_symbol": "ATP9A",
  "gene_name": "Probable phospholipid-transporting ATPase IIA",
  "gene": "UniProtKB:O75110",
  "term_id": "GO:0006890"
}